tRNA(Phe) (7-(3-amino-3-carboxypropyl)wyosine37-C2)-hydroxylase activity [GO:0102524] (molecular function) Sources: GOC:pz, RHEA:37899 Relationships: is a type of 2-oxoglutarate-dependent dioxygenase activity [GO:0016706]; is a type of catalytic activity, acting on a tRNA [GO:0140101] Also known as: tRNAPhe (7-(3-amino-3-carboxypropyl)wyosine37-C2)-hydroxylase activity Definition: Catalysis of the reaction: 2-oxoglutarate + O2 + 7-[(3S)-(3-amino-3-carboxypropyl)]-wyosine37 in tRNAPhe = succinate + carbon dioxide + 7-(2-hydroxy-3-amino-3-carboxypropyl)-wyosine37 in tRNAPhe.